{
  "gene": "UniProtKB:P54253",
  "term_id": "GO:0003723",
  "gene_name": "Ataxin-1",
  "term_label": "RNA binding",
  "gene_symbol": "ATXN1"
}